{
  "gene_symbol": "A0A1W2PRS3",
  "term_label": "transmembrane signaling receptor activity",
  "term_id": "GO:0004888",
  "gene": "UniProtKB:A0A1W2PRS3",
  "gene_name": "Immunoglobulin subtype domain-containing protein"
}